{
  "term_id": "GO:0007169",
  "gene_name": "SHC-transforming protein 3",
  "gene": "UniProtKB:Q92529",
  "term_label": "cell surface receptor protein tyrosine kinase signaling pathway",
  "gene_symbol": "SHC3"
}